negative regulation of retina development in camera-type eye [GO:1902867] (biological process) Also known as: down regulation of retina development in camera-style eye, down regulation of retina development in camera-type eye, down-regulation of retina development in camera-style eye, down-regulation of retina development in camera-type eye, downregulation of retina development in camera-style eye, downregulation of retina development in camera-type eye, negative regulation of retina development in camera-style eye, inhibition of retina development in camera-style eye, inhibition of retina development in camera-type eye, down regulation of retinal development, down-regulation of retinal development, downregulation of retinal development, inhibition of retinal development, negative regulation of retinal development Definition: Any process that stops, prevents or reduces the frequency, rate or extent of retina development in camera-type eye. Relationships: is a type of negative regulation of developmental process [GO:0051093]; is a type of negative regulation of multicellular organismal process [GO:0051241]; is a type of GO:1902866; RO_0002212 GO:0060041 References: PMID:16872597 Sources: GOC:TermGenie, GOC:mr, GO_REF:0000058 Subtypes: GO:0061076